{
  "gene_symbol": "SPCS3",
  "gene_name": "Signal peptidase complex subunit 3",
  "gene": "UniProtKB:P61009",
  "term_id": "GO:0005787",
  "term_label": "signal peptidase complex"
}